germ-band extension [GO:0007377] (BP) Sources: ISBN:0879694238 Definition: Elongation of the germ band on the ventral side of the embryo, accompanied by a halving in width. The elongation process pushes the posterior midgut invagination closed and compresses the amnioserosa further. Relationships: is a type of GO:0048598; is part of gastrulation involving germ band extension [GO:0010004]